{
  "gene_name": "A-kinase anchor protein 5",
  "term_id": "GO:0043197",
  "gene": "UniProtKB:P24588",
  "gene_symbol": "AKAP5",
  "term_label": "dendritic spine"
}